{
  "gene_symbol": "NOC3L",
  "term_label": "chromatin binding",
  "gene_name": "Nucleolar complex protein 3 homolog",
  "gene": "UniProtKB:Q8WTT2",
  "term_id": "GO:0003682"
}